{
  "gene_name": "Sequestosome-1",
  "gene_symbol": "SQSTM1",
  "term_label": "aggresome",
  "term_id": "GO:0016235",
  "gene": "UniProtKB:Q13501"
}